{
  "gene_symbol": "UPK3BL1",
  "gene_name": "Uroplakin-3b-like protein 1",
  "term_id": "UNKNOWN:0001",
  "gene": "UniProtKB:B0FP48",
  "term_label": "Unknown molecular function"
}